{
  "gene_name": "Methionine aminopeptidase 2",
  "gene": "UniProtKB:P50579",
  "gene_symbol": "METAP2",
  "term_id": "GO:0008235",
  "term_label": "metalloexopeptidase activity"
}